{
  "gene": "UniProtKB:Q01151",
  "term_label": "Unknown molecular function",
  "gene_name": "CD83 antigen",
  "gene_symbol": "CD83",
  "term_id": "UNKNOWN:0001"
}